{
  "gene": "UniProtKB:Q96QH8",
  "term_label": "sperm flagellum",
  "gene_symbol": "SPACA5",
  "term_id": "GO:0036126",
  "gene_name": "Sperm acrosome-associated protein 5"
}